{
  "gene_name": "Malectin",
  "gene_symbol": "MLEC",
  "term_id": "UNKNOWN:0001",
  "term_label": "Unknown molecular function",
  "gene": "UniProtKB:Q14165"
}